{
  "term_id": "GO:0021675",
  "term_label": "nerve development",
  "gene_name": "Neurotrophin-3",
  "gene": "UniProtKB:P20783",
  "gene_symbol": "NTF3"
}